cell cycle [GO:0007049] (biological process) Also known as: cell-division cycle Sources: GOC:go_curators, GOC:mtg_cell_cycle Subtypes: mitotic cell cycle [GO:0000278], meiotic cell cycle [GO:0051321] Definition: The progression of biochemical and morphological phases and events that occur in a cell during successive cell replication or nuclear replication events. Canonically, the cell cycle comprises the replication and segregation of genetic material followed by the division of the cell, but in endocycles or syncytial cells nuclear replication or nuclear division may not be followed by cell division. Regulation: negatively regulated by GO:0045786; positively regulated by GO:0045787; regulated by GO:0051726 Relationships: is a type of cellular process [GO:0009987]